{
  "term_id": "GO:0045944",
  "gene_symbol": "RXRA",
  "term_label": "positive regulation of transcription by RNA polymerase II",
  "gene_name": "Retinoic acid receptor RXR-alpha",
  "gene": "UniProtKB:P19793"
}